{
  "term_id": "UNKNOWN:0002",
  "term_label": "Unknown biological process",
  "gene_symbol": "EVC",
  "gene_name": "EvC complex member EVC",
  "gene": "UniProtKB:P57679"
}